{
  "gene_name": "Collagen alpha-1(XXVI) chain",
  "term_id": "UNKNOWN:0002",
  "term_label": "Unknown biological process",
  "gene_symbol": "COL26A1",
  "gene": "UniProtKB:Q96A83"
}